{
  "term_label": "heart contraction",
  "gene": "UniProtKB:Q92629",
  "gene_symbol": "SGCD",
  "term_id": "GO:0060047",
  "gene_name": "Delta-sarcoglycan"
}